{
  "gene": "UniProtKB:Q969D9",
  "gene_symbol": "TSLP",
  "term_label": "positive regulation of interleukin-6 production",
  "term_id": "GO:0032755",
  "gene_name": "Thymic stromal lymphopoietin"
}